regulation of tolerance induction [GO:0002643] (biological process) Definition: Any process that modulates the frequency, rate, or extent of tolerance induction. Relationships: is a type of regulation of immune system process [GO:0002682]; regulates tolerance induction [GO:0002507] Sources: GOC:add Subtypes: negative regulation of tolerance induction [GO:0002644], positive regulation of tolerance induction [GO:0002645], GO:0002646, regulation of tolerance induction to self antigen [GO:0002649], regulation of tolerance induction dependent upon immune response [GO:0002652], regulation of B cell tolerance induction [GO:0002661], regulation of T cell tolerance induction [GO:0002664], regulation of natural killer cell tolerance induction [GO:0002871], regulation of lymphocyte anergy [GO:0002911], regulation of macrophage tolerance induction [GO:0010932]